{
  "term_label": "RNA polymerase II cis-regulatory region sequence-specific DNA binding",
  "term_id": "GO:0000978",
  "gene_name": "Forkhead box protein L1",
  "gene": "UniProtKB:Q12952",
  "gene_symbol": "FOXL1"
}